{
  "gene_name": "Serine_threonine-protein kinase ICK",
  "gene": "UniProtKB:Q9UPZ9",
  "gene_symbol": "CILK1",
  "term_label": "cytoplasm",
  "term_id": "GO:0005737"
}